{
  "gene_symbol": "IGKV5-2",
  "gene": "UniProtKB:P06315",
  "term_id": "GO:0006955",
  "term_label": "immune response",
  "gene_name": "Immunoglobulin kappa variable 5-2"
}